{
  "gene": "UniProtKB:A6NL99",
  "gene_symbol": "AQP7P3",
  "gene_name": "Putative aquaporin-7-like protein 3",
  "term_label": "Unknown biological process",
  "term_id": "UNKNOWN:0002"
}